{
  "gene_symbol": "RPA1",
  "term_id": "GO:0006289",
  "term_label": "nucleotide-excision repair",
  "gene": "UniProtKB:P27694",
  "gene_name": "Replication protein A 70 kDa DNA-binding subunit"
}